{
  "term_label": "protein kinase A binding",
  "term_id": "GO:0051018",
  "gene_name": "A-kinase anchor protein 3",
  "gene": "UniProtKB:O75969",
  "gene_symbol": "AKAP3"
}